{
  "term_id": "UNKNOWN:0001",
  "gene_symbol": "PRXL2C",
  "gene_name": "Peroxiredoxin-like 2C",
  "term_label": "Unknown molecular function",
  "gene": "UniProtKB:Q7RTV5"
}